{
  "gene": "UniProtKB:C9JH25",
  "term_id": "UNKNOWN:0001",
  "gene_name": "Proline-rich transmembrane protein 4",
  "term_label": "Unknown molecular function",
  "gene_symbol": "PRRT4"
}